spore membrane bending pathway [GO:0070583] (biological process) Also known as: FSM bending, ascospore-type prospore membrane bending, forespore membrane bending Definition: The process in which a bending force is generated in the prospore membrane to form the characteristic curved shape of the prospore. References: PMID:18756268 Sources: GOC:dgf Relationships: is_a membrane organization [GO:0061024]; is a type of meiotic cell cycle process [GO:1903046]; is part of ascospore-type prospore membrane formation [GO:0032120]